{
  "gene_symbol": "PSD2",
  "gene_name": "PH and SEC7 domain-containing protein 2",
  "gene": "UniProtKB:Q9BQI7",
  "term_label": "vesicle-mediated transport",
  "term_id": "GO:0016192"
}